{
  "gene": "UniProtKB:P61366",
  "term_label": "extracellular space",
  "gene_symbol": "OSTN",
  "gene_name": "Osteocrin",
  "term_id": "GO:0005615"
}